{
  "term_id": "GO:0005768",
  "gene_symbol": "VPS26A",
  "term_label": "endosome",
  "gene": "UniProtKB:O75436",
  "gene_name": "Vacuolar protein sorting-associated protein 26A"
}